{
  "gene": "UniProtKB:P84095",
  "gene_name": "Rho-related GTP-binding protein RhoG",
  "gene_symbol": "RHOG",
  "term_label": "plasma membrane",
  "term_id": "GO:0005886"
}